{
  "gene_symbol": "TUBA1A",
  "gene": "UniProtKB:Q71U36",
  "term_label": "structural constituent of cytoskeleton",
  "gene_name": "Tubulin alpha-1A chain",
  "term_id": "GO:0005200"
}